intraciliary transport particle A binding [GO:0120160] (molecular function) Definition: Binding to an intraciliary transport particle A (IFT A) complex. References: PMID:20889716 Also known as: intraciliary transport complex A binding, intraflagellar transport complex A binding, intraflagellar transport particle A binding, IFT A complex binding Relationships: is a type of GO:0044877